{
  "gene_name": "Protein odd-skipped-related 2",
  "gene": "UniProtKB:Q8N2R0",
  "term_id": "GO:0000977",
  "term_label": "RNA polymerase II transcription regulatory region sequence-specific DNA binding",
  "gene_symbol": "OSR2"
}